{
  "term_label": "gamma-tubulin ring complex",
  "gene_name": "Mitotic-spindle organizing protein 1",
  "gene": "UniProtKB:Q08AG7",
  "term_id": "GO:0000931",
  "gene_symbol": "MZT1"
}